{
  "gene_symbol": "SCYGR7",
  "gene": "UniProtKB:A0A286YF01",
  "term_id": "UNKNOWN:0002",
  "term_label": "Unknown biological process",
  "gene_name": "Small cysteine and glycine repeat-containing protein 7"
}